{
  "gene": "UniProtKB:Q9C0C2",
  "term_label": "nucleus",
  "gene_name": "182 kDa tankyrase-1-binding protein",
  "term_id": "GO:0005634",
  "gene_symbol": "TNKS1BP1"
}